{
  "gene": "UniProtKB:Q9UHP7",
  "gene_symbol": "CLEC2D",
  "term_label": "NK T cell activation",
  "term_id": "GO:0051132",
  "gene_name": "C-type lectin domain family 2 member D"
}